{
  "gene_symbol": "LMNB2",
  "term_label": "nuclear migration",
  "gene": "UniProtKB:Q03252",
  "term_id": "GO:0007097",
  "gene_name": "Lamin-B2"
}